{
  "term_label": "cytoplasm",
  "term_id": "GO:0005737",
  "gene": "UniProtKB:Q96J87",
  "gene_name": "CUGBP Elav-like family member 6",
  "gene_symbol": "CELF6"
}